{
  "term_id": "GO:0005689",
  "gene": "UniProtKB:Q8TBF4",
  "gene_symbol": "ZCRB1",
  "term_label": "U12-type spliceosomal complex",
  "gene_name": "Zinc finger CCHC-type and RNA-binding motif-containing protein 1"
}